{
  "term_label": "Unknown biological process",
  "gene_symbol": "TRGV8",
  "term_id": "UNKNOWN:0002",
  "gene": "UniProtKB:A0A0C4DH27",
  "gene_name": "T cell receptor gamma variable 8"
}